{
  "gene_symbol": "TGM7",
  "gene": "UniProtKB:Q96PF1",
  "term_label": "protein-glutamine gamma-glutamyltransferase activity",
  "gene_name": "Protein-glutamine gamma-glutamyltransferase Z",
  "term_id": "GO:0003810"
}